AAU codon-amino acid adaptor activity [GO:0033441] (molecular function) Also known as: AAT codon-amino acid adaptor activity, asparagine tRNA Definition: A triplet codon-amino acid adaptor activity that recognizes an AAU codon. Note: Note that in the standard genetic code, AAT codes for asparagine. Sources: GOC:mah Relationships: is a type of GO:0030533